negative energy taxis [GO:0052129] (biological process) Definition: The directed movement of a motile cell or organism towards a lower level of a physical stimulus involved in energy generation, such as light, oxygen, and oxidizable substrates. Sources: GOC:mtg_pamgo_17jul06 Subtypes: negative phototaxis [GO:0046957], negative aerotaxis [GO:0052130] Relationships: is a type of energy taxis [GO:0009453]